{
  "gene": "UniProtKB:Q8N148",
  "gene_name": "Olfactory receptor 6V1",
  "term_label": "plasma membrane",
  "term_id": "GO:0005886",
  "gene_symbol": "OR6V1"
}